{
  "gene_symbol": "MYO7B",
  "gene_name": "Unconventional myosin-VIIb",
  "gene": "UniProtKB:Q6PIF6",
  "term_id": "GO:0015629",
  "term_label": "actin cytoskeleton"
}